{
  "gene": "UniProtKB:Q07912",
  "gene_name": "Activated CDC42 kinase 1",
  "term_label": "protein tyrosine kinase activity",
  "gene_symbol": "TNK2",
  "term_id": "GO:0004713"
}